ionotropic sweet taste receptor activity [GO:0170023] (molecular function) Definition: Enables the transmembrane transfer of an ion by a channel that opens when a specific soluble sweet compound has been bound by the channel complex or one of its constituent parts. Relationships: is a type of ionotropic taste receptor activity [GO:0170021] References: PMID:24474785